{
  "term_id": "GO:0005847",
  "gene_name": "Pre-mRNA 3'-end-processing factor FIP1",
  "term_label": "mRNA cleavage and polyadenylation specificity factor complex",
  "gene_symbol": "FIP1L1",
  "gene": "UniProtKB:Q6UN15"
}